{
  "gene": "UniProtKB:P49411",
  "gene_symbol": "TUFM",
  "term_label": "mitochondrion",
  "term_id": "GO:0005739",
  "gene_name": "Elongation factor Tu, mitochondrial"
}